{
  "gene_symbol": "ACAT1",
  "term_id": "GO:0003985",
  "gene": "UniProtKB:P24752",
  "gene_name": "Acetyl-CoA acetyltransferase, mitochondrial",
  "term_label": "acetyl-CoA C-acetyltransferase activity"
}